{
  "gene_name": "Cornifin-B",
  "gene": "UniProtKB:P22528",
  "term_id": "GO:0001533",
  "term_label": "cornified envelope",
  "gene_symbol": "SPRR1B"
}